{
  "term_label": "ribonucleoprotein complex",
  "gene_name": "CUGBP Elav-like family member 2",
  "gene": "UniProtKB:O95319",
  "gene_symbol": "CELF2",
  "term_id": "GO:1990904"
}